{
  "gene_symbol": "STK33",
  "gene_name": "Serine_threonine-protein kinase 33",
  "gene": "UniProtKB:Q9BYT3",
  "term_label": "nucleus",
  "term_id": "GO:0005634"
}